positive regulation of adaptive immune response based on somatic recombination of immune receptors built from immunoglobulin superfamily domains [GO:0002824] (biological process) Relationships: is a type of GO:0002821; is_a regulation of adaptive immune response based on somatic recombination of immune receptors built from immunoglobulin superfamily domains [GO:0002822]; positively regulates adaptive immune response based on somatic recombination of immune receptors built from immunoglobulin superfamily domains [GO:0002460] Definition: Any process that activates or increases the frequency, rate, or extent of an adaptive immune response based on somatic recombination of immune receptors built from immunoglobulin superfamily domains. An example of this process is found in the Gnathostomata. Subtypes: GO:0002636, positive regulation of tolerance induction dependent upon immune response [GO:0002654], positive regulation of T cell mediated immunity [GO:0002711], positive regulation of B cell mediated immunity [GO:0002714], positive regulation of T-helper 1 type immune response [GO:0002827], GO:0035397, GO:2000318 Sources: GOC:add, GOC:mtg_sensu